mitochondria-nucleus signaling pathway [GO:0031930] (BP) Relationships: is a type of GO:0035556 Definition: The series of molecular signals that forms a pathway of communication from the mitochondria to the nucleus and initiates cellular changes in response to changes in mitochondrial function. References: PMID:15068799 Sources: GOC:jh Also known as: mitochondria-nucleus signal transduction, mitochondrial signaling pathway, mitochondrial signalling pathway, retrograde response